{
  "term_id": "GO:0010468",
  "term_label": "regulation of gene expression",
  "gene": "UniProtKB:Q9Y577",
  "gene_symbol": "TRIM17",
  "gene_name": "E3 ubiquitin-protein ligase TRIM17"
}